{
  "term_label": "mRNA splicing, via spliceosome",
  "gene": "UniProtKB:Q2TBE0",
  "gene_symbol": "CWF19L2",
  "gene_name": "CWF19-like protein 2",
  "term_id": "GO:0000398"
}